{
  "term_label": "Unknown cellular component",
  "term_id": "UNKNOWN:0003",
  "gene_symbol": "SPDYE9",
  "gene": "UniProtKB:A0A494C191",
  "gene_name": "Putative speedy protein E9"
}